{
  "gene": "UniProtKB:Q9H2D1",
  "gene_name": "Mitochondrial folate transporter_carrier",
  "term_id": "GO:0055085",
  "gene_symbol": "SLC25A32",
  "term_label": "transmembrane transport"
}